{
  "term_label": "carbon dioxide transmembrane transport",
  "gene_symbol": "AQP1",
  "gene": "UniProtKB:P29972",
  "gene_name": "Aquaporin-1",
  "term_id": "GO:0035378"
}